{
  "gene_symbol": "ERBB2",
  "term_label": "basal plasma membrane",
  "gene": "UniProtKB:P04626",
  "term_id": "GO:0009925",
  "gene_name": "Receptor tyrosine-protein kinase erbB-2"
}